arginine 2-monooxygenase activity [GO:0047678] (molecular function) Definition: Catalysis of the reaction: L-arginine + O2 = 4-guanidinobutanamide + CO2 + H2O. Also known as: L-arginine:oxygen 2-oxidoreductase (decarboxylating), arginine decarboxy-oxidase activity, arginine monooxygenase activity, arginine oxygenase (decarboxylating) activity Relationships: is a type of oxidoreductase activity, acting on single donors with incorporation of molecular oxygen, incorporation of one atom of oxygen (internal monooxygenases or internal mixed function oxidases) [GO:0016703] Sources: EC:1.13.12.1, RHEA:10548